{
  "gene_name": "Paraneoplastic antigen-like protein 8C",
  "gene_symbol": "PNMA8C",
  "term_label": "Unknown molecular function",
  "gene": "UniProtKB:A0A1B0GUJ8",
  "term_id": "UNKNOWN:0001"
}